bisphosphoglycerate mutase activity [GO:0004082] (molecular function) Definition: Catalysis of the reaction: 3-phospho-D-glyceroyl phosphate = 2,3-bisphospho-D-glycerate. Relationships: is a type of intramolecular phosphotransferase activity [GO:0016868] Also known as: bisphosphoglyceromutase, 2,3-bisphosphoglycerate mutase activity, 2,3-bisphosphoglycerate synthase activity, 2,3-diphosphoglycerate mutase activity, 2,3-diphosphoglycerate synthase activity, 2,3-diphosphoglyceromutase activity, 3-phospho-D-glycerate 1,2-phosphomutase activity, BPGM activity, DPGM, biphosphoglycerate synthase activity, bisphosphoglycerate synthase activity, diphosphoglycerate mutase activity, diphosphoglyceric mutase activity, diphosphoglyceromutase activity, glycerate phosphomutase activity Sources: EC:5.4.2.4